{
  "term_id": "UNKNOWN:0003",
  "gene_symbol": "KCTD9",
  "gene": "UniProtKB:Q7L273",
  "gene_name": "BTB_POZ domain-containing protein KCTD9",
  "term_label": "Unknown cellular component"
}